negative regulation of mitotic telomere tethering at nuclear periphery [GO:1904537] (biological process) Also known as: down regulation of mitotic telomere tethering at nuclear periphery, down-regulation of mitotic telomere tethering at nuclear periphery, downregulation of mitotic telomere tethering at nuclear periphery, inhibition of mitotic telomere tethering at nuclear periphery Relationships: is a type of GO:0048519; is a type of regulation of mitotic telomere tethering at nuclear periphery [GO:1904536]; RO_0002212 mitotic telomere tethering at nuclear periphery [GO:0044820] Definition: Any process that stops, prevents or reduces the frequency, rate or extent of mitotic telomere tethering at nuclear periphery. References: PMID:22959349 Sources: GOC:TermGenie, GO_REF:0000058